trans-Golgi network transport vesicle lumen [GO:0098564] (cellular component) Sources: GOC:dos Relationships: is a type of Golgi lumen [GO:0005796]; is a type of GO:0098566; is part of trans-Golgi network transport vesicle [GO:0030140] Definition: The volume enclosed within the membrane of a trans-Golgi network transport vesicle.